{
  "term_label": "Unknown molecular function",
  "gene_symbol": "IL4",
  "term_id": "UNKNOWN:0001",
  "gene_name": "Interleukin-4",
  "gene": "UniProtKB:P05112"
}